{
  "gene_symbol": "TK1",
  "term_id": "GO:0046104",
  "gene": "UniProtKB:P04183",
  "gene_name": "Thymidine kinase, cytosolic",
  "term_label": "thymidine metabolic process"
}